O6-alkylguanine-DNA binding [GO:0032132] (molecular function) Definition: Binding to an O6-alkylguanine adduct in DNA. References: PMID:16679453 Sources: GOC:mah Relationships: is a type of alkylated DNA binding [GO:0032131]